{
  "term_id": "UNKNOWN:0001",
  "gene": "UniProtKB:Q6ICH7",
  "term_label": "Unknown molecular function",
  "gene_name": "Aspartate beta-hydroxylase domain-containing protein 2",
  "gene_symbol": "ASPHD2"
}